{
  "term_label": "Unknown biological process",
  "gene": "UniProtKB:A0A1B0GVM6",
  "gene_name": "Uncharacterized protein C11orf97",
  "gene_symbol": "C11orf97",
  "term_id": "UNKNOWN:0002"
}